double-stranded miRNA binding [GO:0098851] (molecular function) Relationships: is a type of double-stranded RNA binding [GO:0003725] References: PMID:19966796 Sources: GOC:BHF, GOC:BHF_miRNA, GOC:rph Also known as: miRNA duplex binding Definition: Binding to double-stranded miRNA. double-stranded miRNA is formed by processing of pre-miRNA stem-loop structures.